{
  "term_id": "GO:0008331",
  "term_label": "high voltage-gated calcium channel activity",
  "gene_name": "Voltage-dependent T-type calcium channel subunit alpha-1I",
  "gene": "UniProtKB:Q9P0X4",
  "gene_symbol": "CACNA1I"
}